{
  "term_id": "GO:0001755",
  "gene": "UniProtKB:Q13591",
  "term_label": "neural crest cell migration",
  "gene_name": "Semaphorin-5A",
  "gene_symbol": "SEMA5A"
}